syringetin 7-O-methyltransferase activity [GO:0102441] (molecular function) Sources: RHEA:74735 Definition: Catalysis of the reaction: S-adenosyl-L-methionine + syringetin = 7,3',5'-O-trimethylmyricetin + H+ + S-adenosyl-L-homocysteine. Relationships: is a type of methyltransferase activity [GO:0008168]